{
  "gene": "UniProtKB:Q9Y5G0",
  "gene_name": "Protocadherin gamma-B5",
  "gene_symbol": "PCDHGB5",
  "term_label": "cell adhesion",
  "term_id": "GO:0007155"
}